{
  "gene": "UniProtKB:Q9Y446",
  "term_id": "GO:0005886",
  "term_label": "plasma membrane",
  "gene_symbol": "PKP3",
  "gene_name": "Plakophilin-3"
}